{
  "gene_name": "Heat shock 70 kDa protein 1-like",
  "gene": "UniProtKB:P34931",
  "term_id": "GO:0005886",
  "gene_symbol": "HSPA1L",
  "term_label": "plasma membrane"
}